{
  "gene_symbol": "RBM12B",
  "term_label": "regulation of RNA splicing",
  "gene_name": "RNA-binding protein 12B",
  "gene": "UniProtKB:Q8IXT5",
  "term_id": "GO:0043484"
}